{
  "term_label": "plasma membrane",
  "term_id": "GO:0005886",
  "gene": "UniProtKB:Q9Y5Y4",
  "gene_symbol": "PTGDR2",
  "gene_name": "Prostaglandin D2 receptor 2"
}